{
  "term_id": "GO:0007097",
  "gene_symbol": "SYNE3",
  "gene": "UniProtKB:Q6ZMZ3",
  "term_label": "nuclear migration",
  "gene_name": "Nesprin-3"
}